{
  "gene_name": "Uncharacterized protein",
  "term_id": "GO:0005789",
  "term_label": "endoplasmic reticulum membrane",
  "gene": "UniProtKB:A0A2R8YE69",
  "gene_symbol": "A0A2R8YE69"
}